protein-coenzyme A linkage [GO:0018246] (biological process) Subtypes: GO:0018247 Relationships: is a type of protein modification process [GO:0036211] Sources: GOC:mah Definition: The formation of a linkage between a protein amino acid and coenzyme A.